regulation of DNA recombination at telomere [GO:0072695] (biological process) Subtypes: regulation of telomere maintenance via recombination [GO:0032207], negative regulation of DNA recombination at telomere [GO:0048239], positive regulation of DNA recombination at telomere [GO:0072696] Definition: Any process that modulates the frequency, rate or extent of DNA recombination within the telomere. Also known as: regulation of telomeric recombination Sources: GOC:mah Relationships: is a type of regulation of DNA recombination [GO:0000018]